{
  "gene_name": "Cytochrome c oxidase subunit 7A2, mitochondrial",
  "gene_symbol": "COX7A2",
  "gene": "UniProtKB:P14406",
  "term_label": "protein-macromolecule adaptor activity",
  "term_id": "GO:0030674"
}